{
  "gene_name": "E3 ubiquitin-protein ligase NEDD4",
  "term_id": "GO:0032801",
  "gene_symbol": "NEDD4",
  "term_label": "receptor catabolic process",
  "gene": "UniProtKB:P46934"
}